{
  "gene": "UniProtKB:Q9BY60",
  "term_label": "cellular response to nitrogen starvation",
  "term_id": "GO:0006995",
  "gene_symbol": "GABARAPL3",
  "gene_name": "Gamma-aminobutyric acid receptor-associated protein-like 3"
}